cellular response to cesium ion [GO:0071278] (biological process) Relationships: is a type of response to cesium ion [GO:0010164]; is a type of cellular response to metal ion [GO:0071248] Definition: Any process that results in a change in state or activity of a cell (in terms of movement, secretion, enzyme production, gene expression, etc.) as a result of a cesium stimulus. Also known as: cellular response to cesium Sources: GOC:mah